{
  "term_id": "GO:0043005",
  "gene_symbol": "HTR3B",
  "gene_name": "5-hydroxytryptamine receptor 3B",
  "gene": "UniProtKB:O95264",
  "term_label": "neuron projection"
}